{
  "gene_symbol": "RNASEH2B",
  "gene": "UniProtKB:Q5TBB1",
  "term_id": "GO:0005654",
  "gene_name": "Ribonuclease H2 subunit B",
  "term_label": "nucleoplasm"
}